periplasmic side of cell outer membrane [GO:0031241] (cellular component) Note: In GO, 'internal side' still refers to part of the membrane and does not refer to components beyond (inside of) the membrane. Relationships: is_a GO:0098552; is part of cell outer membrane [GO:0009279] Sources: GOC:mlg, GOC:mtg_sensu Also known as: internal leaflet of cell outer membrane, internal side of cell outer membrane, internal side of outer membrane Definition: The side (leaflet) of the outer membrane that faces the periplasm of the cell.